filamentous growth of a population of unicellular organisms in response to neutral pH [GO:0036178] (biological process) Regulation: regulated by GO:1900440; negatively regulated by negative regulation of filamentous growth of a population of unicellular organisms in response to neutral pH [GO:1900441]; positively regulated by positive regulation of filamentous growth of a population of unicellular organisms in response to neutral pH [GO:1900442] Definition: The process in which a group of unicellular organisms grow in a threadlike, filamentous shape in response to a neutral pH (pH close to 7) stimulus. References: PMID:6374461 Sources: GOC:di Relationships: is_a response to neutral pH [GO:0036176]; is a type of GO:0036177